{
  "gene_symbol": "OR4C11",
  "term_id": "UNKNOWN:0002",
  "gene_name": "Olfactory receptor 4C11",
  "term_label": "Unknown biological process",
  "gene": "UniProtKB:Q6IEV9"
}